{
  "gene_symbol": "ASB12",
  "gene_name": "Ankyrin repeat and SOCS box protein 12",
  "term_label": "ubiquitin ligase complex",
  "term_id": "GO:0000151",
  "gene": "UniProtKB:Q8WXK4"
}